{
  "term_label": "Unknown biological process",
  "gene_symbol": "MTG2",
  "term_id": "UNKNOWN:0002",
  "gene_name": "Mitochondrial ribosome-associated GTPase 2",
  "gene": "UniProtKB:Q9H4K7"
}